{
  "gene_name": "Phospholipase A and acyltransferase 1",
  "term_id": "GO:0004623",
  "term_label": "phospholipase A2 activity",
  "gene": "UniProtKB:Q9HDD0",
  "gene_symbol": "PLAAT1"
}